{
  "gene": "UniProtKB:Q9UPY8",
  "term_label": "regulation of microtubule polymerization or depolymerization",
  "term_id": "GO:0031110",
  "gene_symbol": "MAPRE3",
  "gene_name": "Microtubule-associated protein RP_EB family member 3"
}